{
  "gene": "UniProtKB:P61081",
  "gene_name": "NEDD8-conjugating enzyme Ubc12",
  "gene_symbol": "UBE2M",
  "term_label": "nucleus",
  "term_id": "GO:0005634"
}